{
  "term_id": "GO:0000978",
  "gene_symbol": "GLI1",
  "gene_name": "Zinc finger protein GLI1",
  "gene": "UniProtKB:P08151",
  "term_label": "RNA polymerase II cis-regulatory region sequence-specific DNA binding"
}